negative regulation of N-terminal peptidyl-methionine acetylation [GO:1904664] (biological process) References: PMID:20807799 Sources: GOC:TermGenie, GO_REF:0000058 Relationships: is a type of negative regulation of protein acetylation [GO:1901984]; is a type of negative regulation of protein maturation [GO:1903318]; is a type of regulation of N-terminal peptidyl-methionine acetylation [GO:1904663]; negatively regulates N-terminal peptidyl-methionine acetylation [GO:0017196] Definition: Any process that stops, prevents or reduces the frequency, rate or extent of N-terminal peptidyl-methionine acetylation.